{
  "gene": "UniProtKB:Q8NI77",
  "term_id": "GO:0008574",
  "gene_name": "Kinesin-like protein KIF18A",
  "term_label": "plus-end-directed microtubule motor activity",
  "gene_symbol": "KIF18A"
}